{
  "gene": "UniProtKB:Q5JQD4",
  "gene_name": "Putative peptide YY-3",
  "gene_symbol": "PYY3",
  "term_id": "GO:0005615",
  "term_label": "extracellular space"
}